{
  "gene_name": "Maestro heat-like repeat-containing protein family member 7",
  "term_id": "UNKNOWN:0002",
  "gene": "UniProtKB:Q68CQ1",
  "term_label": "Unknown biological process",
  "gene_symbol": "MROH7"
}